{
  "gene": "UniProtKB:Q9Y6D5",
  "gene_name": "Brefeldin A-inhibited guanine nucleotide-exchange protein 2",
  "term_label": "trans-Golgi network",
  "gene_symbol": "ARFGEF2",
  "term_id": "GO:0005802"
}